{
  "term_label": "negative regulation of transforming growth factor beta receptor signaling pathway",
  "gene": "UniProtKB:Q14392",
  "gene_symbol": "LRRC32",
  "term_id": "GO:0030512",
  "gene_name": "Transforming growth factor beta activator LRRC32"
}